phosphonoacetate hydrolase activity [GO:0047400] (molecular function) Relationships: is a type of hydrolase activity, acting on acid carbon-phosphorus bonds [GO:0016827] Definition: Catalysis of the reaction: H2O + phosphonoacetate = acetate + H+ + phosphate. Also known as: phosphonoacetate phosphonohydrolase activity Sources: RHEA:16749